regulation of formation by symbiont of haustorium for nutrient acquisition from host [GO:0075045] (biological process) Note: Note that this term should not be used to annotate gene products of the host. It should only be used to annotate those gene products from the symbiont involved in this process. Subtypes: GO:0075046, negative regulation of formation by symbiont of haustorium for nutrient acquisition from host [GO:0075047] Relationships: is a type of GO:0022603; is a type of regulation of biological process involved in symbiotic interaction [GO:0043903]; is a type of modulation of formation of structure involved in a symbiotic process [GO:0044145]; regulates formation of haustorium for nutrient acquisition [GO:0052094] Definition: Any process that modulates the frequency, rate or extent of symbiont haustorium formation for nutrient acquisition from host. The host is defined as the larger of the organisms involved in a symbiotic interaction. Sources: GOC:pamgo_curators